{
  "term_label": "extracellular space",
  "term_id": "GO:0005615",
  "gene": "UniProtKB:P14151",
  "gene_name": "L-selectin",
  "gene_symbol": "SELL"
}